{
  "gene_symbol": "TOMM40L",
  "gene": "UniProtKB:Q969M1",
  "term_id": "GO:0008320",
  "gene_name": "Mitochondrial import receptor subunit TOM40B",
  "term_label": "protein transmembrane transporter activity"
}